DNA-templated transcriptional start site selection [GO:0001173] (biological process) Subtypes: transcriptional start site selection at RNA polymerase II promoter [GO:0001174], transcriptional start site selection at RNA polymerase III promoter [GO:0001175] Also known as: DNA-dependent transcriptional start site selection, transcriptional start site selection at bacterial-type RNA polymerase promoter Definition: Any process involved in the selection of the specific location within the template strand of a DNA-dependent RNA polymerase promoter for hybridization of the cognate ribonucleotides and formation of first phosphodiester bond within the nascent transcript. Relationships: is a type of RNA biosynthetic process [GO:0032774]; is part of DNA-templated transcription initiation [GO:0006352] References: PMID:16826228, PMID:18846104 Sources: GOC:txnOH